{
  "gene": "UniProtKB:Q86UU5",
  "gene_name": "Gametogenetin",
  "term_id": "GO:0031625",
  "gene_symbol": "GGN",
  "term_label": "ubiquitin protein ligase binding"
}